{
  "gene_symbol": "CDH11",
  "term_label": "adherens junction",
  "term_id": "GO:0005912",
  "gene": "UniProtKB:P55287",
  "gene_name": "Cadherin-11"
}